{
  "term_label": "Golgi vesicle docking",
  "term_id": "GO:0048211",
  "gene_symbol": "USO1",
  "gene": "UniProtKB:O60763",
  "gene_name": "General vesicular transport factor p115"
}